{
  "term_label": "Unknown biological process",
  "gene_name": "Nitric oxide synthase-interacting protein",
  "gene": "UniProtKB:Q9Y314",
  "gene_symbol": "NOSIP",
  "term_id": "UNKNOWN:0002"
}